{
  "gene_name": "Growth-regulated alpha protein",
  "gene_symbol": "CXCL1",
  "gene": "UniProtKB:P09341",
  "term_label": "Unknown molecular function",
  "term_id": "UNKNOWN:0001"
}